{
  "gene": "UniProtKB:P17301",
  "term_label": "integrin-mediated signaling pathway",
  "gene_symbol": "ITGA2",
  "term_id": "GO:0007229",
  "gene_name": "Integrin alpha-2"
}